{
  "term_id": "GO:0005739",
  "term_label": "mitochondrion",
  "gene": "UniProtKB:O14561",
  "gene_symbol": "NDUFAB1",
  "gene_name": "Acyl carrier protein, mitochondrial"
}